{
  "gene_symbol": "CBX2",
  "gene": "UniProtKB:Q14781",
  "term_id": "GO:0062072",
  "term_label": "histone H3K9me2/3 reader activity",
  "gene_name": "Chromobox protein homolog 2"
}